negative regulation of somatic muscle development [GO:0062225] (biological process) Relationships: is_a negative regulation of developmental process [GO:0051093]; is a type of regulation of somatic muscle development [GO:0062223]; negatively regulates somatic muscle development [GO:0007525] References: PMID:16643882, PMID:25758712 Subtypes: negative regulation of adult somatic muscle development [GO:0062228], negative regulation of larval somatic muscle development [GO:0062230] Definition: Any process that decreases the rate, frequency or extent of somatic muscle development.